{
  "term_id": "GO:0140693",
  "gene_symbol": "G3BP2",
  "gene_name": "Ras GTPase-activating protein-binding protein 2",
  "term_label": "molecular condensate scaffold activity",
  "gene": "UniProtKB:Q9UN86"
}